{
  "gene": "UniProtKB:Q96PX8",
  "gene_symbol": "SLITRK1",
  "gene_name": "SLIT and NTRK-like protein 1",
  "term_label": "GABA-ergic synapse",
  "term_id": "GO:0098982"
}